positive regulation of synaptonemal complex assembly [GO:1905088] (BP) Relationships: is a type of GO:0044089; is a type of GO:0090068; is a type of GO:0090173; is a type of positive regulation of reproductive process [GO:2000243]; is a type of positive regulation of chromosome organization [GO:2001252]; positively regulates GO:0007130 References: PMID:24797370 Sources: GOC:TermGenie, GO_REF:0000058 Also known as: positive regulation of synaptonemal complex formation, up regulation of synaptonemal complex assembly, up regulation of synaptonemal complex formation, up-regulation of synaptonemal complex assembly, up-regulation of synaptonemal complex formation, upregulation of synaptonemal complex assembly, upregulation of synaptonemal complex formation, activation of synaptonemal complex assembly, activation of synaptonemal complex formation Definition: Any process that activates or increases the frequency, rate or extent of synaptonemal complex assembly.